{
  "gene": "UniProtKB:O94829",
  "gene_name": "Importin-13",
  "gene_symbol": "IPO13",
  "term_label": "cytoplasm",
  "term_id": "GO:0005737"
}